{
  "gene": "UniProtKB:Q8WXR4",
  "gene_name": "Myosin-IIIb",
  "term_id": "GO:0001917",
  "gene_symbol": "MYO3B",
  "term_label": "photoreceptor inner segment"
}